{
  "term_id": "GO:0030515",
  "term_label": "snoRNA binding",
  "gene": "UniProtKB:Q9H583",
  "gene_symbol": "HEATR1",
  "gene_name": "HEAT repeat-containing protein 1"
}